positive regulation of selenocysteine incorporation [GO:1904571] (biological process) Definition: Any process that activates or increases the frequency, rate or extent of selenocysteine incorporation. Relationships: is_a positive regulation of translational elongation [GO:0045901]; is a type of GO:1904569; positively regulates selenocysteine incorporation [GO:0001514] Also known as: up regulation of selenocysteine incorporation, up-regulation of selenocysteine incorporation, upregulation of selenocysteine incorporation, activation of selenocysteine incorporation References: PMID:21685449 Sources: GOC:TermGenie, GO_REF:0000058